{
  "gene_symbol": "LANCL1",
  "term_id": "GO:0004364",
  "gene_name": "Glutathione S-transferase LANCL1",
  "gene": "UniProtKB:O43813",
  "term_label": "glutathione transferase activity"
}